{
  "term_label": "Unknown cellular component",
  "gene": "UniProtKB:Q96R54",
  "term_id": "UNKNOWN:0003",
  "gene_name": "Olfactory receptor 14A2",
  "gene_symbol": "OR14A2"
}